regulation of aldosterone secretion [GO:2000858] (biological process) Relationships: is a type of regulation of mineralocorticoid secretion [GO:2000855]; regulates aldosterone secretion [GO:0035932] Sources: GOC:sl Definition: Any process that modulates the frequency, rate or extent of aldosterone secretion. Subtypes: renin-angiotensin regulation of aldosterone production [GO:0002018], GO:2000859, positive regulation of aldosterone secretion [GO:2000860]